{
  "term_id": "GO:0005912",
  "gene_symbol": "MSN",
  "gene": "UniProtKB:P26038",
  "term_label": "adherens junction",
  "gene_name": "Moesin"
}